basal pole of neuron [GO:0044226] (cellular component) Sources: NIF_Subcellular:sao1186862860 Definition: Portion of a neuron cell soma closest to the point where the basilar dendrite emerges. Relationships: is a type of cell pole [GO:0060187]; is part of neuronal cell body [GO:0043025]